{
  "gene_name": "Keratin, type I cuticular Ha3-II",
  "term_id": "GO:0045109",
  "gene_symbol": "KRT33B",
  "term_label": "intermediate filament organization",
  "gene": "UniProtKB:Q14525"
}